{
  "gene_name": "Alpha-tectorin",
  "term_label": "extracellular matrix structural constituent",
  "term_id": "GO:0005201",
  "gene_symbol": "TECTA",
  "gene": "UniProtKB:O75443"
}